salicylic acid glucosyltransferase (glucoside-forming) activity [GO:0052640] (MF) Also known as: salicylic acid glucosyltransferase activity, UDP:glucose:2-hydroxybenzoic acid glucosyltransferase (glucoside-forming) activity, UDP:glucose:SA glucosyltransferase (glucoside-forming) activity, UDP:glucose:salicylate glucosyltransferase (glucoside-forming) activity, UDP:glucose:salicylic acid glucosyltransferase (glucoside-forming) activity Relationships: is a type of UDP-glucosyltransferase activity [GO:0035251] Definition: Catalysis of the reaction: salicylic acid + UDP-glucose = salicylic acid 2-O-glucoside + UDP. Sources: MetaCyc:RXN-11658, RHEA:62312